{
  "gene": "UniProtKB:O95837",
  "term_label": "cytoplasm",
  "gene_name": "Guanine nucleotide-binding protein subunit alpha-14",
  "gene_symbol": "GNA14",
  "term_id": "GO:0005737"
}